{
  "gene_symbol": "NMRAL1",
  "gene_name": "NmrA-like family domain-containing protein 1",
  "term_id": "UNKNOWN:0001",
  "term_label": "Unknown molecular function",
  "gene": "UniProtKB:Q9HBL8"
}